hexose metabolic process [GO:0019318] (biological process) Definition: The chemical reactions and pathways involving a hexose, any monosaccharide with a chain of six carbon atoms in the molecule. Sources: ISBN:0198506732 Also known as: hexose metabolism Relationships: is a type of monosaccharide metabolic process [GO:0005996] Subtypes: fructose metabolic process [GO:0006000], GO:0006004, glucose metabolic process [GO:0006006], GO:0006012, mannose metabolic process [GO:0006013], hexose biosynthetic process [GO:0019319], hexose catabolic process [GO:0019320]